scattered antral spaces stage [GO:0048163] (biological process) Definition: The stage in oogenesis when antral spaces begin to form in the follicle cells. Mitochondria form centers for yolk concentration. Sources: GOC:jid, GOC:mtg_sensu, ISBN:0198542771 Also known as: mammalian oogenesis stage 6 Relationships: is a type of mammalian oogenesis stage [GO:0022605]